{
  "term_label": "AMP kinase activity",
  "term_id": "GO:0004017",
  "gene": "UniProtKB:Q96M32",
  "gene_name": "Adenylate kinase 7",
  "gene_symbol": "AK7"
}